{
  "term_label": "mitochondrial outer membrane translocase complex assembly",
  "gene_symbol": "MTX3",
  "gene_name": "Metaxin-3",
  "gene": "UniProtKB:Q5HYI7",
  "term_id": "GO:0070096"
}